pyrimidine nucleotide salvage [GO:0032262] (BP) Sources: GOC:mah Relationships: is a type of GO:0006221; is a type of pyrimidine-containing compound salvage [GO:0008655]; is a type of GO:0043173 Definition: Any process which produces a pyrimidine nucleotide from derivatives of it, without de novo synthesis. Subtypes: pyrimidine ribonucleotide salvage [GO:0010138], pyrimidine deoxyribonucleotide salvage [GO:0010139]